{
  "gene": "UniProtKB:P04626",
  "gene_name": "Receptor tyrosine-protein kinase erbB-2",
  "gene_symbol": "ERBB2",
  "term_label": "positive regulation of MAPK cascade",
  "term_id": "GO:0043410"
}